{
  "gene_name": "Ankyrin repeat domain-containing protein 42",
  "term_label": "cyclin-dependent protein serine/threonine kinase inhibitor activity",
  "gene_symbol": "ANKRD42",
  "gene": "UniProtKB:Q8N9B4",
  "term_id": "GO:0004861"
}